channel regulator activity [GO:0016247] (molecular function) Subtypes: GO:0016248, GO:0099103, ion channel regulator activity [GO:0099106] Sources: GOC:mah Definition: Binds to and modulates the activity of a channel. A channel catalyzes energy-independent facilitated diffusion, mediated by passage of a solute through a transmembrane aqueous pore or channel. Relationships: is a type of transporter regulator activity [GO:0141108]; RO_0002211 channel activity [GO:0015267]